{
  "term_label": "respiratory chain complex III",
  "gene_symbol": "MT-CYB",
  "gene": "UniProtKB:P00156",
  "gene_name": "Cytochrome b",
  "term_id": "GO:0045275"
}